{
  "term_id": "GO:0000977",
  "gene": "UniProtKB:O14627",
  "term_label": "RNA polymerase II transcription regulatory region sequence-specific DNA binding",
  "gene_name": "Homeobox protein CDX-4",
  "gene_symbol": "CDX4"
}